{
  "gene_symbol": "BRINP1",
  "term_label": "dendrite",
  "gene": "UniProtKB:O60477",
  "term_id": "GO:0030425",
  "gene_name": "BMP_retinoic acid-inducible neural-specific protein 1"
}